negative regulation of extracellular matrix disassembly [GO:0010716] (biological process) Also known as: down regulation of extracellular matrix disassembly, down-regulation of extracellular matrix disassembly, downregulation of extracellular matrix disassembly, negative regulation of extracellular matrix breakdown, negative regulation of extracellular matrix degradation, inhibition of extracellular matrix disassembly Sources: GOC:BHF, GOC:dph, GOC:tb Definition: Any process that decreases the rate, frequency or extent of extracellular matrix disassembly. Extracellular matrix disassembly is a process that results in the breakdown of the extracellular matrix. Relationships: is a type of regulation of extracellular matrix disassembly [GO:0010715]; is a type of negative regulation of extracellular matrix organization [GO:1903054]; negatively regulates GO:0022617